{
  "gene_symbol": "FGF16",
  "gene_name": "Fibroblast growth factor 16",
  "term_id": "GO:0022008",
  "gene": "UniProtKB:O43320",
  "term_label": "neurogenesis"
}